alphav-beta5 integrin-osteopontin complex [GO:0070031] (cellular component) Definition: A protein complex that consists of an alphav-beta5 integrin complex bound to osteopontin. References: PMID:7592829 Also known as: ITGAV-ITGB5-SPP1 complex Relationships: is a type of plasma membrane protein complex [GO:0098797]